P-type zinc transporter activity [GO:0016463] (molecular function) Definition: Enables the transfer of a solute or solutes from one side of a membrane to the other according to the reaction: ATP + H2O + Zn2+(in) = ADP + phosphate + Zn2+(out). Sources: RHEA:20621 Also known as: zinc exporting ATPase activity, ATP phosphohydrolase (Zn2+-exporting), zinc-translocating P-type ATPase activity, P(1B)-type ATPase activity, P1B-type ATPase activity, Zn(2+)-exporting ATPase activity, Zn2+-exporting ATPase activity, zinc transmembrane transporter activity, phosphorylative mechanism, zinc-exporting ATPase activity Relationships: is_a zinc ion transmembrane transporter activity [GO:0005385]; is a type of P-type ion transporter activity [GO:0015662]; is_a ATPase-coupled monoatomic cation transmembrane transporter activity [GO:0019829]